mucus secretion [GO:0070254] (biological process) Also known as: mucus production Relationships: is a type of body fluid secretion [GO:0007589]; is a type of GO:0032941 Sources: GOC:add, ISBN:068340007X, ISBN:0721662544 Regulation: regulated by regulation of mucus secretion [GO:0070255]; negatively regulated by GO:0070256; positively regulated by positive regulation of mucus secretion [GO:0070257] Definition: The regulated release of mucus by the mucosa. Mucus is a viscous slimy secretion consisting of mucins and various inorganic salts dissolved in water, with suspended epithelial cells and leukocytes. The mucosa, or mucous membrane, is the membrane covered with epithelium that lines the tubular organs of the body. Mucins are carbohydrate-rich glycoproteins that have a lubricating and protective function.